uniplex complex [GO:1990246] (cellular component) References: PMID:24231807 Definition: A calcium channel complex in the mitochondrial inner membrane capable of highly-selective calcium channel activity. Its components include the EF-hand-containing proteins mitochondrial calcium uptake 1 (MICU1) and MICU2, the pore-forming subunit mitochondrial calcium uniporter (MCU) and its paralog MCUb, and the MCU regulator EMRE. Relationships: is_a GO:0034704; is_a inner mitochondrial membrane protein complex [GO:0098800] Also known as: mitochondrial uniporter complex, mitochondrial uniporter holocomplex